TSC1-TSC2 complex binding [GO:0062078] (molecular function) Also known as: tuberin sclerosis complex binding, tuberin-hamartin complex binding Relationships: is a type of GO:0044877 References: PMID:28561066 Definition: Binding to a TSC1-TSC2 complex.